{
  "gene_name": "Unconventional myosin-VI",
  "term_id": "GO:0001726",
  "gene": "UniProtKB:Q9UM54",
  "gene_symbol": "MYO6",
  "term_label": "ruffle"
}